positive regulation of larval salivary gland boundary specification [GO:0045712] (biological process) Relationships: is a type of positive regulation of salivary gland boundary specification [GO:0045706]; is a type of regulation of larval salivary gland boundary specification [GO:0045708]; positively regulates larval salivary gland boundary specification [GO:0007433] Also known as: positive regulation of larval salivary gland determination, up regulation of larval salivary gland determination, up-regulation of larval salivary gland determination, upregulation of larval salivary gland determination, activation of larval salivary gland determination, stimulation of larval salivary gland determination Sources: GOC:go_curators, GOC:tb Definition: Any process that activates or increases the frequency, rate or extent of salivary gland determination in a larval organism.